positive regulation of sensory neuron axon guidance [GO:1905491] (BP) Definition: Any process that activates or increases the frequency, rate or extent of sensory neuron axon guidance. References: PMID:16516839 Sources: GOC:TermGenie, GO_REF:0000058 Also known as: up regulation of sensory neuron axon guidance, up-regulation of sensory neuron axon guidance, upregulation of sensory neuron axon guidance, activation of sensory neuron axon guidance Relationships: is_a positive regulation of axon guidance [GO:1902669]; is a type of GO:1905489; positively regulates sensory neuron axon guidance [GO:0097374]